UDP-galacturonate decarboxylase activity [GO:0050374] (molecular function) Definition: Catalysis of the reaction: H+ + UDP-alpha-D-galacturonate = CO2 + UDP-L-arabinose. Sources: EC:4.1.1.67, RHEA:19725 Also known as: UDP-D-galacturonate carboxy-lyase (UDP-L-arabinose-forming), UDP-D-galacturonate carboxy-lyase activity, UDP-galacturonic acid decarboxylase activity, UDPGalUA carboxy lyase activity, UDPgalacturonate decarboxylase activity Relationships: is a type of GO:0016831